{
  "gene": "UniProtKB:P01567",
  "gene_name": "Interferon alpha-7",
  "term_id": "GO:0005132",
  "gene_symbol": "IFNA7",
  "term_label": "type I interferon receptor binding"
}